{
  "gene_name": "Proton-coupled amino acid transporter 3",
  "gene": "UniProtKB:Q495N2",
  "term_label": "L-alanine transmembrane transporter activity",
  "term_id": "GO:0015180",
  "gene_symbol": "SLC36A3"
}